{
  "term_id": "UNKNOWN:0001",
  "gene": "UniProtKB:A8MZH6",
  "term_label": "Unknown molecular function",
  "gene_symbol": "OOSP1",
  "gene_name": "Putative oocyte-secreted protein 1 homolog"
}